{
  "gene": "UniProtKB:P01127",
  "term_id": "GO:0070374",
  "gene_symbol": "PDGFB",
  "term_label": "positive regulation of ERK1 and ERK2 cascade",
  "gene_name": "Platelet-derived growth factor subunit B"
}